{
  "gene_name": "Protein lin-52 homolog",
  "gene": "UniProtKB:Q52LA3",
  "term_id": "UNKNOWN:0002",
  "gene_symbol": "LIN52",
  "term_label": "Unknown biological process"
}